{
  "term_label": "cytoplasm",
  "gene_name": "Kelch-like protein 6",
  "gene_symbol": "KLHL6",
  "term_id": "GO:0005737",
  "gene": "UniProtKB:Q8WZ60"
}